{
  "gene_name": "5-formyltetrahydrofolate cyclo-ligase",
  "term_id": "GO:0035999",
  "gene_symbol": "MTHFS",
  "gene": "UniProtKB:P49914",
  "term_label": "tetrahydrofolate interconversion"
}